positive regulation of collateral sprouting of intact axon in response to injury [GO:0048684] (biological process) Sources: GOC:dgh, GOC:dph, GOC:jid, GOC:lm Definition: Any process that activates, maintains or increases the rate of collateral sprouting of an intact axon as a result of injury to an axon. Also known as: up regulation of collateral sprouting of intact axon in response to injury, up-regulation of collateral sprouting of intact axon in response to injury, upregulation of collateral sprouting of intact axon in response to injury, activation of collateral sprouting of intact axon in response to injury, stimulation of collateral sprouting of intact axon in response to injury Relationships: is a type of positive regulation of collateral sprouting [GO:0048672]; is_a positive regulation of axon regeneration [GO:0048680]; is a type of regulation of collateral sprouting of intact axon in response to injury [GO:0048683]; positively regulates collateral sprouting of intact axon in response to injury [GO:0048673]